{
  "term_label": "autophagosome assembly",
  "term_id": "GO:0000045",
  "gene": "UniProtKB:Q86TL0",
  "gene_symbol": "ATG4D",
  "gene_name": "Cysteine protease ATG4D"
}